{
  "gene_name": "Catenin alpha-2",
  "term_id": "GO:0098609",
  "gene_symbol": "CTNNA2",
  "term_label": "cell-cell adhesion",
  "gene": "UniProtKB:P26232"
}